{
  "gene": "UniProtKB:Q8N3Z0",
  "term_id": "UNKNOWN:0002",
  "gene_symbol": "PRSS35",
  "gene_name": "Inactive serine protease 35",
  "term_label": "Unknown biological process"
}